{
  "gene_name": "Cytochrome P450 4F11",
  "term_id": "GO:0042376",
  "term_label": "phylloquinone catabolic process",
  "gene": "UniProtKB:Q9HBI6",
  "gene_symbol": "CYP4F11"
}